{
  "gene_name": "Integrator complex subunit 1",
  "term_label": "Unknown molecular function",
  "term_id": "UNKNOWN:0001",
  "gene": "UniProtKB:Q8N201",
  "gene_symbol": "INTS1"
}